nuclear aryl hydrocarbon receptor complex [GO:0034753] (cellular component) Definition: An aryl hydrocarbon receptor (AhR) complex found in the nucleus; ; consists of ligand-bound AhR and the aryl hydrocarbon receptor nuclear translocator (ARNT). Relationships: is a type of aryl hydrocarbon receptor complex [GO:0034751]; is a type of GO:0140513 References: PMID:7598497 Also known as: nuclear AHRC, nuclear AhR complex, 6S-nuclear aryl hydrocarbon (Ah) receptor ligand-activated complex